isoamylase activity [GO:0019156] (MF) Relationships: is_a GO:0004553 Also known as: debranching enzyme activity, glycogen alpha-1,6-glucanohydrolase activity Sources: EC:3.2.1.68 Definition: Catalysis of the hydrolysis of alpha-(1,6)-D-glucosidic branch linkages in glycogen, amylopectin and their beta-limits dextrins.